{
  "gene": "UniProtKB:A0A0A0MRZ8",
  "gene_symbol": "IGKV3D-11",
  "term_id": "UNKNOWN:0001",
  "gene_name": "Immunoglobulin kappa variable 3D-11",
  "term_label": "Unknown molecular function"
}